photoreceptor activity [GO:0009881] (molecular function) Sources: GOC:ai, GOC:go_curators Definition: The function of absorbing and responding to incidental electromagnetic radiation, particularly visible light. The response may involve a change in conformation. Also known as: UV-sensitive opsin, blue-sensitive opsin, green-sensitive opsin, long-wave-sensitive opsin, opsin, red-sensitive opsin, short-wave-sensitive opsin, violet-sensitive opsin Relationships: is a type of signaling receptor activity [GO:0038023] Subtypes: G protein-coupled photoreceptor activity [GO:0008020], GO:0009882, red or far-red light photoreceptor activity [GO:0009883]